phospholipase activator activity [GO:0016004] (molecular function) Definition: Binds to and increases the activity of a phospholipase, an enzyme that catalyzes of the hydrolysis of a glycerophospholipid. Subtypes: GO:0016005, sphingomyelin phosphodiesterase activator activity [GO:0016230], phospholipase C activator activity [GO:0160185], phospholipase D activator activity [GO:1990583] Sources: GOC:ai Relationships: is a type of lipase activator activity [GO:0060229]; positively regulates phospholipase activity [GO:0004620]